{
  "gene_name": "pre-rRNA 2'-O-ribose RNA methyltransferase FTSJ3",
  "term_id": "GO:0000466",
  "term_label": "maturation of 5.8S rRNA from tricistronic rRNA transcript (SSU-rRNA, 5.8S rRNA, LSU-rRNA)",
  "gene_symbol": "FTSJ3",
  "gene": "UniProtKB:Q8IY81"
}